{
  "gene": "UniProtKB:Q9Y219",
  "term_label": "Unknown cellular component",
  "gene_name": "Protein jagged-2",
  "gene_symbol": "JAG2",
  "term_id": "UNKNOWN:0003"
}